{
  "gene_name": "Electron transfer flavoprotein subunit alpha, mitochondrial",
  "gene": "UniProtKB:P13804",
  "gene_symbol": "ETFA",
  "term_id": "GO:0005739",
  "term_label": "mitochondrion"
}